{
  "gene_name": "Hepatocyte nuclear factor 3-gamma",
  "term_label": "RNA polymerase II cis-regulatory region sequence-specific DNA binding",
  "term_id": "GO:0000978",
  "gene_symbol": "FOXA3",
  "gene": "UniProtKB:P55318"
}